malonyl-CoA biosynthetic process [GO:2001295] (BP) Definition: The chemical reactions and pathways resulting in the formation of malonyl-CoA, the S-malonyl derivative of coenzyme A. Relationships: is a type of acyl-CoA biosynthetic process [GO:0071616]; is a type of malonyl-CoA metabolic process [GO:2001293] Also known as: malonyl-CoA anabolism, malonyl-CoA biosynthesis, malonyl-CoA formation, malonyl-CoA synthesis Sources: GOC:yaf, UniPathway:UPA00655